positive regulation of inflammatory response to wounding [GO:0106016] (BP) Definition: Any process that activates or increases the frequency, rate or extent of the inflammatory response to wounding. References: PMID:26022821 Sources: GOC:BHF, GOC:BHF_miRNA, GOC:rph Relationships: is a type of GO:0050729; is a type of regulation of inflammatory response to wounding [GO:0106014]; is a type of positive regulation of response to wounding [GO:1903036]; positively regulates inflammatory response to wounding [GO:0090594]